negative regulation of fibronectin-dependent thymocyte migration [GO:2000414] (biological process) Definition: Any process that stops, prevents or reduces the frequency, rate or extent of fibronectin-dependent thymocyte migration. Sources: GOC:BHF, GOC:mah Also known as: negative regulation of fibronectin-dependent thymic lymphocyte migration, negative regulation of fibronectin-dependent immature T cell migration, negative regulation of fibronectin-dependent immature T lymphocyte migration, negative regulation of fibronectin-dependent immature T-cell migration, negative regulation of fibronectin-dependent immature T-lymphocyte migration Relationships: is a type of negative regulation of thymocyte migration [GO:2000411]; is a type of regulation of fibronectin-dependent thymocyte migration [GO:2000413]; negatively regulates fibronectin-dependent thymocyte migration [GO:0072681]